{
  "gene_symbol": "AKAP8L",
  "term_label": "nucleus",
  "term_id": "GO:0005634",
  "gene_name": "A-kinase anchor protein 8-like",
  "gene": "UniProtKB:Q9ULX6"
}